{
  "gene_symbol": "SIAE",
  "gene_name": "Sialate O-acetylesterase",
  "term_id": "UNKNOWN:0003",
  "gene": "UniProtKB:Q9HAT2",
  "term_label": "Unknown cellular component"
}